{
  "term_label": "sensory perception of sound",
  "gene_symbol": "TMIE",
  "gene_name": "Transmembrane inner ear expressed protein",
  "gene": "UniProtKB:Q8NEW7",
  "term_id": "GO:0007605"
}